{
  "gene": "UniProtKB:P13765",
  "term_label": "lysosomal membrane",
  "gene_symbol": "HLA-DOB",
  "term_id": "GO:0005765",
  "gene_name": "HLA class II histocompatibility antigen, DO beta chain"
}